{
  "gene": "UniProtKB:P20962",
  "gene_symbol": "PTMS",
  "gene_name": "Parathymosin",
  "term_label": "histone binding",
  "term_id": "GO:0042393"
}